{
  "term_id": "GO:0003924",
  "gene_name": "Ras-related protein Rap-1b",
  "gene_symbol": "RAP1B",
  "gene": "UniProtKB:P61224",
  "term_label": "GTPase activity"
}